{
  "gene_symbol": "PELI3",
  "term_id": "UNKNOWN:0003",
  "gene": "UniProtKB:Q8N2H9",
  "term_label": "Unknown cellular component",
  "gene_name": "E3 ubiquitin-protein ligase pellino homolog 3"
}